{
  "gene_symbol": "ZNF70",
  "term_id": "GO:0000981",
  "gene": "UniProtKB:Q9UC06",
  "term_label": "DNA-binding transcription factor activity, RNA polymerase II-specific",
  "gene_name": "Zinc finger protein 70"
}